{
  "gene_name": "RAB7A-interacting MON1-CCZ1 complex subunit 1",
  "gene_symbol": "RIMOC1",
  "gene": "UniProtKB:A6NDU8",
  "term_id": "UNKNOWN:0001",
  "term_label": "Unknown molecular function"
}